hexosaminidase activity [GO:0015929] (molecular function) Sources: ISBN:0721662544 Relationships: is a type of hydrolase activity, hydrolyzing O-glycosyl compounds [GO:0004553] Subtypes: N-acetylglucosamine-1-phosphodiester alpha-N-acetylglucosaminidase activity [GO:0003944], GO:0004415, alpha-N-acetylglucosaminidase activity [GO:0004561], GO:0004563, alpha-N-acetylgalactosaminidase activity [GO:0008456], endogalactosaminidase activity [GO:0033931], GO:0052774, GO:0061784 Definition: Catalysis of the cleavage of hexosamine or N-acetylhexosamine residues (e.g. N-acetylglucosamine) residues from gangliosides or other glycoside oligosaccharides.